regulation of release of sequestered calcium ion into cytosol [GO:0051279] (biological process) Definition: Any process that modulates the frequency, rate or extent of the release into the cytosolic compartment of calcium ions sequestered in the endoplasmic reticulum or mitochondria. Relationships: is a type of regulation of sequestering of calcium ion [GO:0051282]; is_a regulation of calcium ion transmembrane transport [GO:1903169]; regulates release of sequestered calcium ion into cytosol [GO:0051209] Also known as: regulation of release of sequestered calcium ion (Ca2+), regulation of release of stored calcium ion (Ca2+), regulation of calcium ion (Ca2+) mobilization, regulation of calcium mobilization, regulation of cytoplasmic release of sequestered calcium ion (Ca2+), regulation of cytoplasmic release of stored calcium ion (Ca2+), regulation of release of stored calcium ion (Ca2+) into cytoplasm, regulation of release of stored calcium ion (Ca2+) into cytosol Subtypes: regulation of release of sequestered calcium ion into cytosol by sarcoplasmic reticulum [GO:0010880], GO:0051280, positive regulation of release of sequestered calcium ion into cytosol [GO:0051281], regulation of ryanodine-sensitive calcium-release channel activity [GO:0060314], regulation of Golgi calcium ion export [GO:1901472] Sources: GOC:ai, GOC:tb